establishment of planar polarity [GO:0001736] (biological process) Subtypes: establishment of imaginal disc-derived wing hair orientation [GO:0001737], establishment of cell polarity involved in growth plate cartilage chondrocyte division [GO:0003424], establishment of ommatidial planar polarity [GO:0042067], GO:0042247, establishment of planar polarity of embryonic epithelium [GO:0042249], establishment of planar polarity of larval imaginal disc epithelium [GO:0042252], establishment of body hair or bristle planar orientation [GO:0048104], establishment of planar polarity involved in nephron morphogenesis [GO:0072046] Regulation: regulated by regulation of establishment of planar polarity [GO:0090175] Definition: Coordinated organization of groups of cells in the plane of an epithelium, such that they all orient to similar coordinates. Sources: GOC:dph Also known as: establishment of planar cell polarity Relationships: is a type of establishment of tissue polarity [GO:0007164]; is part of GO:0001738